{
  "term_label": "regulation of transcription by RNA polymerase II",
  "gene": "UniProtKB:O43309",
  "gene_symbol": "ZSCAN12",
  "term_id": "GO:0006357",
  "gene_name": "Zinc finger and SCAN domain-containing protein 12"
}